{
  "gene_symbol": "ERVK13-1",
  "term_id": "UNKNOWN:0002",
  "gene": "UniProtKB:Q9NX77",
  "term_label": "Unknown biological process",
  "gene_name": "Endogenous retrovirus group K member 13-1 Env polyprotein"
}